{
  "gene": "UniProtKB:P62701",
  "term_label": "structural constituent of ribosome",
  "gene_symbol": "RPS4X",
  "term_id": "GO:0003735",
  "gene_name": "Small ribosomal subunit protein eS4, X isoform"
}